GDP-mannose:serine-protein mannose-1-phosphotransferase activity [GO:0018422] (molecular function) Definition: Catalysis of the transfer of mannose-1-phosphate to a serine residue in a protein. Relationships: is a type of GO:0016780 References: PMID:10037765 Sources: GOC:mah